{
  "term_id": "GO:0005737",
  "gene_name": "Cytochrome P450 2A13",
  "term_label": "cytoplasm",
  "gene": "UniProtKB:Q16696",
  "gene_symbol": "CYP2A13"
}